{
  "gene": "UniProtKB:Q9H0C2",
  "term_id": "GO:0046902",
  "gene_symbol": "SLC25A31",
  "gene_name": "ADP_ATP translocase 4",
  "term_label": "regulation of mitochondrial membrane permeability"
}